mitotic spindle assembly [GO:0090307] (BP) Relationships: is a type of mitotic spindle organization [GO:0007052]; is a type of spindle assembly [GO:0051225]; is part of GO:0000070 Also known as: spindle assembly involved in mitosis Sources: GOC:tb, GOC:vw Definition: Mitotic bipolar spindle assembly begins with spindle microtubule nucleation from the separated spindle pole body, includes spindle elongation during prometaphase, and is complete when all kinetochores are stably attached the spindle, and the spindle assembly checkpoint is satisfied. Regulation: regulated by regulation of mitotic spindle assembly [GO:1901673] Subtypes: mitotic spindle formation (spindle phase two) [GO:0140641]